{
  "term_label": "cell surface receptor signaling pathway via JAK-STAT",
  "gene_name": "Signal transducer and activator of transcription 5B",
  "gene": "UniProtKB:P51692",
  "term_id": "GO:0007259",
  "gene_symbol": "STAT5B"
}